{
  "gene": "UniProtKB:Q9BY78",
  "gene_symbol": "RNF26",
  "gene_name": "E3 ubiquitin-protein ligase RNF26",
  "term_id": "GO:0016567",
  "term_label": "protein ubiquitination"
}